{
  "gene_symbol": "SLC13A1",
  "gene_name": "Solute carrier family 13 member 1",
  "gene": "UniProtKB:Q9BZW2",
  "term_id": "GO:0005886",
  "term_label": "plasma membrane"
}